{
  "term_label": "Unknown biological process",
  "term_id": "UNKNOWN:0002",
  "gene_symbol": "IQANK1",
  "gene_name": "IQ motif and ankyrin repeat domain-containing protein 1",
  "gene": "UniProtKB:A8MXQ7"
}